positive regulation of salicylic acid mediated signaling pathway [GO:0080151] (biological process) References: PMID:20181750 Definition: Any process that activates or increases the frequency, rate or extent of salicylic acid mediated signal transduction. Relationships: is a type of positive regulation of signal transduction [GO:0009967]; is a type of regulation of salicylic acid mediated signaling pathway [GO:2000031]; positively regulates salicylic acid mediated signaling pathway [GO:0009863] Also known as: positive regulation of salicylic acid mediated signalling pathway